{
  "gene_name": "Transmembrane protein 225B",
  "term_id": "UNKNOWN:0002",
  "gene": "UniProtKB:P0DP42",
  "gene_symbol": "TMEM225B",
  "term_label": "Unknown biological process"
}